{
  "gene": "UniProtKB:Q13033",
  "gene_symbol": "STRN3",
  "term_id": "GO:0030674",
  "term_label": "protein-macromolecule adaptor activity",
  "gene_name": "Striatin-3"
}